npBAF complex [GO:0071564] (cellular component) Relationships: is a type of SWI/SNF superfamily-type complex [GO:0070603] References: PMID:17640523 Sources: GOC:mah, GOC:ss Definition: A SWI/SNF-type complex that is found in neural stem or progenitor cells, and in human contains actin and proteins encoded by the ARID1A/BAF250A or ARID1B/BAF250B, SMARCD1/BAF60A, SMARCD3/BAF60C, SMARCA2/BRM/BAF190B, SMARCA4/BRG1/BAF190A, SMARCB1/BAF47, SMARCC1/BAF155, SMARCE1/BAF57, SMARCC2/BAF170, PHF10/BAF45A, ACTL6A/BAF53A genes. The npBAF complex is essential for the self-renewal/proliferative capacity of the multipotent neural stem cells.